{
  "gene_symbol": "LARGE2",
  "gene": "UniProtKB:Q8N3Y3",
  "term_label": "glucuronosyltransferase activity",
  "term_id": "GO:0015020",
  "gene_name": "Xylosyl- and glucuronyltransferase LARGE2"
}